{
  "term_label": "positive regulation of G2/MI transition of meiotic cell cycle",
  "gene": "UniProtKB:P30305",
  "gene_name": "M-phase inducer phosphatase 2",
  "term_id": "GO:0110032",
  "gene_symbol": "CDC25B"
}